palmitoleoyltransferase activity [GO:1990698] (MF) References: PMID:17141155, PMID:25731175 Relationships: is a type of acyltransferase activity, transferring groups other than amino-acyl groups [GO:0016747] Note: Note that this term should not be confused with 'palmitoyltransferase activity ; GO:0016409'. Definition: Catalysis of the transfer of a palmitoleoyl group, a 16-carbon monounsaturated fatty acid (C16:1), to an acceptor molecule.